protein-pyridoxal-5-phosphate linkage via peptidyl-N6-pyridoxal phosphate-L-lysine [GO:0018272] (biological process) Sources: RESID:AA0119 Relationships: is a type of GO:0018205; is a type of protein-pyridoxal-5-phosphate linkage [GO:0018352] Definition: The modification of peptidyl-lysine to form N6-pyridoxal phosphate-L-lysine.